{
  "gene_name": "Tubulin-specific chaperone D",
  "term_label": "GTPase activator activity",
  "gene_symbol": "TBCD",
  "term_id": "GO:0005096",
  "gene": "UniProtKB:Q9BTW9"
}